{
  "term_label": "neuronal cell body membrane",
  "gene_name": "Sodium-dependent noradrenaline transporter",
  "term_id": "GO:0032809",
  "gene": "UniProtKB:P23975",
  "gene_symbol": "SLC6A2"
}